{
  "gene_name": "Olfactory receptor 56A3",
  "term_label": "plasma membrane",
  "gene": "UniProtKB:Q8NH54",
  "gene_symbol": "OR56A3",
  "term_id": "GO:0005886"
}